{
  "term_label": "protein processing",
  "gene_name": "Carboxypeptidase M",
  "gene_symbol": "CPM",
  "term_id": "GO:0016485",
  "gene": "UniProtKB:P14384"
}